chromosome localization [GO:0050000] (biological process) Subtypes: homologous chromosome orientation in meiotic metaphase I [GO:0031619], telomere localization [GO:0034397], GO:0051305, GO:0051310, chromosome localization to nuclear envelope involved in homologous chromosome segregation [GO:0090220], chromosome attachment to the nuclear envelope [GO:0097240], centromere clustering [GO:0098653], GO:0099606, spindle pole body-led chromosome movement during mitotic interphase [GO:0140405], mitotic metaphase chromosome recapture [GO:1990942] Definition: Any process in which a chromosome is transported to, or maintained in, a specific location. Sources: GOC:ai Also known as: chromosome localisation, establishment and maintenance of chromosome localization, establishment and maintenance of chromosome position Relationships: is a type of GO:0051640